regulation of dephosphorylation [GO:0035303] (biological process) Definition: Any process that modulates the frequency, rate or extent of removal of phosphate groups from a molecule. Sources: GOC:bf Relationships: is a type of regulation of phosphorus metabolic process [GO:0051174]; regulates dephosphorylation [GO:0016311] Subtypes: regulation of phosphatase activity [GO:0010921], negative regulation of dephosphorylation [GO:0035305], positive regulation of dephosphorylation [GO:0035306], regulation of phosphatidylinositol dephosphorylation [GO:0060304]